histone mRNA catabolic process [GO:0071044] (biological process) Relationships: is a type of nuclear-transcribed mRNA catabolic process [GO:0000956]; is a type of histone mRNA metabolic process [GO:0008334] Subtypes: GO:0071045 References: PMID:17179095, PMID:17855393 Sources: GOC:dgf, GOC:krc Definition: The chemical reactions and pathways resulting in the breakdown of histone messenger RNA (mRNA).